{
  "gene": "UniProtKB:Q96A57",
  "gene_symbol": "TMEM230",
  "gene_name": "Transmembrane protein 230",
  "term_label": "synaptic vesicle transport",
  "term_id": "GO:0048489"
}